{
  "gene_symbol": "TAS2R16",
  "term_label": "bitter taste receptor activity",
  "gene": "UniProtKB:Q9NYV7",
  "term_id": "GO:0033038",
  "gene_name": "Taste receptor type 2 member 16"
}